negative regulation of phosphorelay signal transduction system [GO:0070298] (biological process) Sources: GOC:mah Relationships: is a type of GO:0070297; is a type of negative regulation of intracellular signal transduction [GO:1902532]; negatively regulates phosphorelay signal transduction system [GO:0000160] Also known as: down regulation of two-component signal transduction, down-regulation of two-component signal transduction, downregulation of two-component signal transduction, negative regulation of histidyl-aspartyl phosphorelay, inhibition of two-component signal transduction, negative regulation of two-component signal transduction system (phosphorelay) Definition: Any process that stops, prevents, or reduces the frequency, rate or extent of signal transduction via a phosphorelay signal transduction system. Subtypes: GO:0010105